negative regulation of interleukin-6 production [GO:0032715] (BP) Sources: GOC:mah Definition: Any process that stops, prevents, or reduces the frequency, rate, or extent of interleukin-6 production. Also known as: down regulation of interleukin-6 production, down-regulation of interleukin-6 production, downregulation of interleukin-6 production, negative regulation of IL-6 production, inhibition of interleukin-6 production, negative regulation of interleukin-6 biosynthetic process, negative regulation of interleukin-6 secretion Relationships: is a type of GO:0001818; is a type of GO:0032675; negatively regulates interleukin-6 production [GO:0032635]